{
  "gene_name": "Olfactory receptor 2AG2",
  "term_label": "olfactory receptor activity",
  "term_id": "GO:0004984",
  "gene_symbol": "OR2AG2",
  "gene": "UniProtKB:A6NM03"
}